{
  "gene_name": "Cytokine-dependent hematopoietic cell linker",
  "gene_symbol": "CLNK",
  "gene": "UniProtKB:Q7Z7G1",
  "term_label": "cell surface receptor protein tyrosine kinase signaling pathway",
  "term_id": "GO:0007169"
}